{
  "gene_name": "Cytochrome P450 7B1",
  "term_id": "GO:0008395",
  "gene": "UniProtKB:O75881",
  "gene_symbol": "CYP7B1",
  "term_label": "steroid hydroxylase activity"
}